mitotic sister chromatid cohesion, arms [GO:0071961] (biological process) Also known as: mitotic sister chromatid cohesion along arms, sister chromatid cohesion along arms at mitosis Sources: GOC:mah Relationships: is a type of mitotic sister chromatid cohesion [GO:0007064] Definition: The cell cycle process in which the sister chromatids of a replicated chromosome are joined along the length of the chromosome arms during mitosis.